lens development in camera-type eye [GO:0002088] (biological process) Relationships: is a type of anatomical structure development [GO:0048856]; is part of GO:0043010 Sources: GOC:dph, ISBN:0582064333 Also known as: lens development, lens development in camera-style eye Definition: The process whose specific outcome is the progression of the lens over time, from its formation to the mature structure. The lens is a transparent structure in the eye through which light is focused onto the retina. An example of this process is found in Mus musculus.